{
  "term_label": "Golgi apparatus",
  "term_id": "GO:0005794",
  "gene_symbol": "SLC35E3",
  "gene_name": "Solute carrier family 35 member E3",
  "gene": "UniProtKB:Q7Z769"
}